transcription elongation-coupled chromatin remodeling [GO:0140673] (biological process) References: PMID:22922743, PMID:28053344 Also known as: co-transcriptional chromatin reassembly, euchromatin maintenance during transcription elongation, maintenance of chromatin integrity during transcription elongation by RNAPII, maintenance of transcriptionally active chromatin during transcription elongation, transcription elongation coupled chromatin remodeling, transcriptional elongation-coupled chromatin remodeling, DNA replication-independent chromatin organization, chromatin maintenance during transcription elongation Definition: A chromatin remodeling process that reestablishes the chromatin structure following the passage of RNA polymerase II during transcription elongation, thus preventing cryptic transcription initiation. Relationships: is_a GO:0006338; is part of transcription elongation by RNA polymerase II [GO:0006368] Note: Note: Do not confuse with 'GO:0045815 transcriptional initiation-coupled chromatin remodeling', which describes the maintenance of chromatin in an open conformation, allowing the transcriptional machinery to access the DNA.